regulation of T-helper 2 cell cytokine production [GO:2000551] (BP) Subtypes: negative regulation of T-helper 2 cell cytokine production [GO:2000552], positive regulation of T-helper 2 cell cytokine production [GO:2000553] Definition: Any process that modulates the frequency, rate or extent of T-helper 2 cell cytokine production. Sources: GOC:obol Also known as: regulation of Th2 cell cytokine production Relationships: is_a regulation of T cell cytokine production [GO:0002724]; is a type of regulation of type 2 immune response [GO:0002828]; regulates T-helper 2 cell cytokine production [GO:0035745]